{
  "gene_name": "AP-3 complex subunit mu-1",
  "gene_symbol": "AP3M1",
  "term_label": "endocytosis",
  "term_id": "GO:0006897",
  "gene": "UniProtKB:Q9Y2T2"
}